{
  "term_id": "GO:1903094",
  "gene_name": "UBX domain-containing protein 1",
  "term_label": "negative regulation of protein K48-linked deubiquitination",
  "gene_symbol": "UBXN1",
  "gene": "UniProtKB:Q04323"
}